{
  "gene_name": "U8 snoRNA-decapping enzyme",
  "term_label": "mRNA catabolic process",
  "term_id": "GO:0006402",
  "gene": "UniProtKB:Q96DE0",
  "gene_symbol": "NUDT16"
}